{
  "term_label": "oncostatin-M receptor activity",
  "gene_symbol": "LIFR",
  "term_id": "GO:0004924",
  "gene_name": "Leukemia inhibitory factor receptor",
  "gene": "UniProtKB:P42702"
}